{
  "term_label": "plasma membrane",
  "term_id": "GO:0005886",
  "gene": "UniProtKB:Q96LC7",
  "gene_name": "Sialic acid-binding Ig-like lectin 10",
  "gene_symbol": "SIGLEC10"
}